{
  "gene": "UniProtKB:Q9UKL0",
  "gene_symbol": "RCOR1",
  "term_id": "GO:0005667",
  "term_label": "transcription regulator complex",
  "gene_name": "REST corepressor 1"
}